{
  "gene_symbol": "IL23A",
  "gene": "UniProtKB:Q9NPF7",
  "term_id": "UNKNOWN:0001",
  "gene_name": "Interleukin-23 subunit alpha",
  "term_label": "Unknown molecular function"
}